{
  "term_label": "voltage-gated proton channel activity",
  "gene": "UniProtKB:Q96D96",
  "gene_name": "Voltage-gated hydrogen channel 1",
  "gene_symbol": "HVCN1",
  "term_id": "GO:0030171"
}